{
  "term_label": "endoplasmic reticulum",
  "term_id": "GO:0005783",
  "gene": "UniProtKB:Q8WTX9",
  "gene_name": "Palmitoyltransferase ZDHHC1",
  "gene_symbol": "ZDHHC1"
}